{
  "gene_name": "Inactive pancreatic lipase-related protein 1",
  "term_id": "GO:0008970",
  "term_label": "phospholipase A1 activity",
  "gene": "UniProtKB:P54315",
  "gene_symbol": "PNLIPRP1"
}